photosystem I stabilization [GO:0042550] (biological process) Definition: The stabilization of the photosystem I protein complex, resulting from the phosphorylation of its structural protein subunits, in a cell actively involved in photosynthesis. Relationships: is a type of regulation of photosynthesis, light reaction [GO:0042548] Sources: GOC:go_curators